positive regulation of protein insertion into mitochondrial outer membrane [GO:1903638] (biological process) Relationships: is a type of positive regulation of organelle organization [GO:0010638]; is a type of regulation of protein insertion into mitochondrial outer membrane [GO:1903636]; is a type of positive regulation of protein targeting to mitochondrion [GO:1903955]; positively regulates protein insertion into mitochondrial outer membrane [GO:0045040] Also known as: positive regulation of mitochondrial outer membrane protein import, positive regulation of protein import into mitochondrial outer membrane, positive regulation of protein transport into mitochondrial outer membrane, up regulation of mitochondrial outer membrane protein import, up regulation of protein import into mitochondrial outer membrane, up regulation of protein insertion into mitochondrial outer membrane, up regulation of protein transport into mitochondrial outer membrane, up-regulation of mitochondrial outer membrane protein import, up-regulation of protein import into mitochondrial outer membrane, up-regulation of protein insertion into mitochondrial outer membrane, up-regulation of protein transport into mitochondrial outer membrane, upregulation of mitochondrial outer membrane protein import, upregulation of protein import into mitochondrial outer membrane, upregulation of protein insertion into mitochondrial outer membrane, upregulation of protein transport into mitochondrial outer membrane, activation of mitochondrial outer membrane protein import, activation of protein import into mitochondrial outer membrane, activation of protein insertion into mitochondrial outer membrane, activation of protein transport into mitochondrial outer membrane Definition: Any process that activates or increases the frequency, rate or extent of protein insertion into mitochondrial outer membrane. References: PMID:16374546 Sources: GOC:TermGenie, GO_REF:0000058